{
  "gene_symbol": "GNGT1",
  "gene": "UniProtKB:P63211",
  "term_id": "GO:0005834",
  "term_label": "heterotrimeric G-protein complex",
  "gene_name": "Guanine nucleotide-binding protein G(T) subunit gamma-T1"
}